cohesin complex [GO:0008278] (cellular component) Also known as: SMC/kleisin ring complex, 14S cohesin, 9S cohesin, Smc1-Smc3 complex, SMC complex, cohesin core heterodimer, nuclear cohesin complex Definition: A protein complex that is required for sister chromatid cohesion in eukaryotes. The cohesin complex forms a molecular ring complex, and is composed of structural maintenance of chromosomes (SMC) and kleisin proteins. For example, in yeast, the complex is composed of the SMC proteins Smc1p and Smc3p, and the kleisin protein Scc1p. In vertebrates, the complex is composed of the SMC1 (SMC1A or SMC1B) and SMC3 heterodimer attached via their hinge domains to a kleisin (RAD21, REC8 or RAD21L) which links them, and one STAG protein (STAG1, STAG2 or STAG3). Relationships: is a type of protein-containing complex [GO:0032991]; is part of chromosome [GO:0005694] References: PMID:9887095 Sources: GOC:jl, GOC:sp, GOC:vw Subtypes: mitotic cohesin complex [GO:0030892], GO:0030893